{
  "gene_name": "Protein Wnt-10b",
  "gene_symbol": "WNT10B",
  "gene": "UniProtKB:O00744",
  "term_id": "GO:0045165",
  "term_label": "cell fate commitment"
}